complement receptor activity [GO:0004875] (molecular function) Definition: Combining with any component or product of the complement cascade and transmitting the signal from one side of the membrane to the other to initiate a change in cell activity. References: PMID:11884446 Sources: GOC:add, GOC:ai, GOC:pg, GOC:signaling, ISBN:0781735149 Also known as: anaphylatoxin receptor activity Note: Note that the complement cascade includes all of the components involved in the classical complement pathway, the alternative complement pathway, and the lectin complement pathway, as well as the common components of all three pathways. Relationships: is_a GO:0004888; is a type of immune receptor activity [GO:0140375]; is part of complement receptor mediated signaling pathway [GO:0002430]; has part GO:0001848 Subtypes: GO:0001857, complement component iC3b receptor activity [GO:0001858], GO:0001859, complement component C3d receptor activity [GO:0001860], complement component C4b receptor activity [GO:0001861], complement component C3a receptor activity [GO:0004876], complement component C3b receptor activity [GO:0004877], GO:0004878